{
  "term_label": "F-actin capping protein complex",
  "gene": "UniProtKB:P47755",
  "term_id": "GO:0008290",
  "gene_name": "F-actin-capping protein subunit alpha-2",
  "gene_symbol": "CAPZA2"
}